{
  "gene": "UniProtKB:O75398",
  "gene_symbol": "DEAF1",
  "term_id": "GO:0005634",
  "term_label": "nucleus",
  "gene_name": "Deformed epidermal autoregulatory factor 1 homolog"
}